{
  "gene_name": "Multiple epidermal growth factor-like domains protein 8",
  "term_id": "GO:0060972",
  "gene_symbol": "MEGF8",
  "gene": "UniProtKB:Q7Z7M0",
  "term_label": "left/right pattern formation"
}